mitochondrial chromosome [GO:0000262] (cellular component) Sources: GOC:mah Definition: A chromosome found in the mitochondrion of a eukaryotic cell. Relationships: is a type of chromosome [GO:0005694]; is part of mitochondrial nucleoid [GO:0042645] Also known as: mitochondrial DNA, mtDNA, mitochondrial genome